olfactory receptor activity [GO:0004984] (molecular function) Relationships: is_a GO:0004888; is part of GO:0050911 References: PMID:19135896, PMID:21041441 Sources: GOC:bf, GOC:dph, GOC:sart Definition: Combining with an odorant and transmitting the signal from one side of the membrane to the other to initiate a change in cell activity in response to detection of smell. Also known as: odorant receptor activity Subtypes: G protein-coupled olfactory receptor activity [GO:0038022], ionotropic olfactory receptor activity [GO:0170020]